{
  "term_label": "extracellular space",
  "term_id": "GO:0005615",
  "gene": "UniProtKB:P58166",
  "gene_symbol": "INHBE",
  "gene_name": "Inhibin beta E chain"
}